{
  "gene": "UniProtKB:Q96T54",
  "term_id": "GO:0071805",
  "term_label": "potassium ion transmembrane transport",
  "gene_name": "Potassium channel subfamily K member 17",
  "gene_symbol": "KCNK17"
}